embryonic liver development [GO:1990402] (biological process) Definition: The process occurring during the embryonic phase whose specific outcome is the progression of the liver over time, from its formation to the mature structure. References: PMID:15918910 Relationships: is a type of GO:0048568